{
  "gene_name": "UDP-glucose:glycoprotein glucosyltransferase 1",
  "gene_symbol": "UGGT1",
  "term_label": "UDP-glucose:glycoprotein glucosyltransferase activity",
  "gene": "UniProtKB:Q9NYU2",
  "term_id": "GO:0003980"
}